{
  "term_label": "quinone reductase (NADPH) activity",
  "gene_symbol": "CRYZ",
  "gene_name": "Quinone oxidoreductase",
  "gene": "UniProtKB:Q08257",
  "term_id": "GO:0003960"
}